fluorene catabolic process [GO:0019429] (biological process) Relationships: is a type of xenobiotic catabolic process [GO:0042178]; is a type of hydrocarbon catabolic process [GO:0120253] References: PMID:15317800 Also known as: fluorene breakdown, fluorene catabolism, fluorene degradation, fluorene metabolism, fluorene metabolic process Definition: The chemical reactions and pathways resulting in the breakdown of fluorene, a tricyclic polycyclic aromatic hydrocarbon containing a five-membered ring. It is a major component of fossil fuels and their derivatives and is also a by-product of coal-conversion and energy-related industries. It is commonly found in vehicle exhaust emissions, crude oils, motor oils, coal and oil combustion products, waste incineration, and industrial effluents.